endocytic vesicle lumen [GO:0071682] (CC) Definition: The volume enclosed by the membrane of an endocytic vesicle. Sources: GOC:pde Subtypes: phagocytic vesicle lumen [GO:0097013], clathrin-coated endocytic vesicle lumen [GO:0106176] Relationships: is a type of intracellular organelle lumen [GO:0070013]; BFO_0000050 endocytic vesicle [GO:0030139]